positive regulation of interleukin-4-mediated signaling pathway [GO:1902216] (biological process) Relationships: is a type of positive regulation of cytokine-mediated signaling pathway [GO:0001961]; is a type of regulation of interleukin-4-mediated signaling pathway [GO:1902214]; positively regulates GO:0035771 References: PMID:17210636 Sources: GOC:TermGenie Definition: Any process that activates or increases the frequency, rate or extent of interleukin-4-mediated signaling pathway. Also known as: positive regulation of IL-4-mediated signaling pathway, positive regulation of interleukin-4-mediated signalling pathway, up regulation of IL-4-mediated signaling pathway, up regulation of interleukin-4-mediated signaling pathway, up regulation of interleukin-4-mediated signalling pathway, up-regulation of IL-4-mediated signaling pathway, up-regulation of interleukin-4-mediated signaling pathway, up-regulation of interleukin-4-mediated signalling pathway, upregulation of IL-4-mediated signaling pathway, upregulation of interleukin-4-mediated signaling pathway, upregulation of interleukin-4-mediated signalling pathway, activation of IL-4-mediated signaling pathway, activation of interleukin-4-mediated signaling pathway, activation of interleukin-4-mediated signalling pathway